lung smooth muscle development [GO:0061145] (biological process) Relationships: is a type of smooth muscle tissue development [GO:0048745]; is part of lung development [GO:0030324] Definition: The process whose specific outcome is the progression of smooth muscle in the lung over time, from its formation to the mature structure. Sources: GOC:dph